{
  "gene_symbol": "DGKZ",
  "gene_name": "Diacylglycerol kinase zeta",
  "term_label": "intracellular signal transduction",
  "term_id": "GO:0035556",
  "gene": "UniProtKB:Q13574"
}